{
  "gene": "UniProtKB:Q9P2U7",
  "term_label": "L-glutamate transmembrane transporter activity",
  "gene_name": "Vesicular glutamate transporter 1",
  "term_id": "GO:0005313",
  "gene_symbol": "SLC17A7"
}